{
  "term_id": "UNKNOWN:0001",
  "term_label": "Unknown molecular function",
  "gene": "UniProtKB:Q6ZTZ1",
  "gene_name": "Myb_SANT-like DNA-binding domain-containing protein 1",
  "gene_symbol": "MSANTD1"
}